seed trichome differentiation [GO:0090376] (biological process) Relationships: is a type of developmental process involved in reproduction [GO:0003006]; is a type of trichome differentiation [GO:0010026]; is a type of cellular process involved in reproduction in multicellular organism [GO:0022412]; is part of seed development [GO:0048316] References: PMID:17905721 Sources: GOC:tb Also known as: seed hair differentiation, cotton fiber development, seed trichome development Definition: The process in which a relatively unspecialized epidermal cell acquires the specialized features of a seed trichome. A seed trichome is a trichome that develops from seed coat epidermis and is often long with putative dispersal function.